phosphoenolpyruvate-glycerone phosphotransferase activity [GO:0047324] (molecular function) Also known as: phosphoenolpyruvate:glycerone phosphotransferase activity Relationships: is_a kinase activity [GO:0016301]; is a type of phosphotransferase activity, alcohol group as acceptor [GO:0016773] Definition: Catalysis of the reaction: glycerone + phosphoenolpyruvate = glycerone phosphate + pyruvate. Sources: EC:2.7.1.121, RHEA:18381